{
  "gene_name": "Tumor necrosis factor alpha-induced protein 3",
  "gene": "UniProtKB:P21580",
  "term_label": "negative regulation of innate immune response",
  "gene_symbol": "TNFAIP3",
  "term_id": "GO:0045824"
}